negative regulation of mitochondrial translational elongation [GO:1905083] (biological process) Also known as: down regulation of mitochondrial translation elongation, down regulation of mitochondrial translational elongation, down-regulation of mitochondrial translation elongation, down-regulation of mitochondrial translational elongation, downregulation of mitochondrial translation elongation, downregulation of mitochondrial translational elongation, negative regulation of mitochondrial translation elongation, inhibition of mitochondrial translation elongation, inhibition of mitochondrial translational elongation Relationships: is a type of negative regulation of translational elongation [GO:0045900]; is a type of GO:0070130; is a type of regulation of mitochondrial translational elongation [GO:1905082]; negatively regulates GO:0070125 Definition: Any process that stops, prevents or reduces the frequency, rate or extent of mitochondrial translational elongation. References: PMID:25738458 Sources: GOC:TermGenie, GO_REF:0000058